cobalamin 5'-phosphate synthase activity [GO:0008818] (molecular function) Definition: Catalysis of the reaction: adenosylcobinamide-GDP + alpha-ribazole-5'-phosphate = adenosylcobalamin-5'-phosphate + GMP. Relationships: is a type of GO:0016780 Sources: MetaCyc:COBALAMIN5PSYN-RXN